{
  "term_id": "GO:0000030",
  "term_label": "mannosyltransferase activity",
  "gene_symbol": "PIGM",
  "gene": "UniProtKB:Q9H3S5",
  "gene_name": "GPI mannosyltransferase 1"
}